{
  "gene": "UniProtKB:Q86TX2",
  "term_label": "fatty acyl-CoA hydrolase activity",
  "term_id": "GO:0047617",
  "gene_name": "Acyl-coenzyme A thioesterase 1",
  "gene_symbol": "ACOT1"
}